{
  "gene_name": "Dapper homolog 1",
  "term_label": "cytoplasm",
  "gene": "UniProtKB:Q9NYF0",
  "term_id": "GO:0005737",
  "gene_symbol": "DACT1"
}